{
  "term_id": "GO:0016024",
  "gene": "UniProtKB:Q96BW9",
  "term_label": "CDP-diacylglycerol biosynthetic process",
  "gene_symbol": "TAMM41",
  "gene_name": "Phosphatidate cytidylyltransferase, mitochondrial"
}